{
  "term_label": "nuclear-transcribed mRNA catabolic process, nonsense-mediated decay",
  "term_id": "GO:0000184",
  "gene": "UniProtKB:Q92540",
  "gene_symbol": "SMG7",
  "gene_name": "Nonsense-mediated mRNA decay factor SMG7"
}